regulation of viral life cycle [GO:1903900] (BP) Definition: Any process that modulates the frequency, rate or extent of viral life cycle. References: PMID:18005716 Sources: GOC:TermGenie, GO_REF:0000058 Also known as: regulation of viral assembly, maturation, egress, and release, regulation of lytic viral life cycle, regulation of viral infectious cycle, regulation of viral replication Relationships: is a type of regulation of viral process [GO:0050792]; RO_0002211 viral life cycle [GO:0019058] Subtypes: regulation of viral genome replication [GO:0045069], regulation of viral entry into host cell [GO:0046596], GO:1901252, regulation of receptor-mediated virion attachment to host cell [GO:1902734], GO:1903901, GO:1903902, regulation of viral DNA genome packaging via site-specific sequence recognition [GO:1905137]